{
  "term_label": "Unknown molecular function",
  "gene_name": "T cell receptor alpha chain constant",
  "gene": "UniProtKB:P01848",
  "gene_symbol": "TRAC",
  "term_id": "UNKNOWN:0001"
}